symbiont-mediated perturbation of host opsonization [GO:0141073] (biological process) Definition: A process in which a symbiont alters or subverts opsonization by the host. The host is defined as the larger of the organisms involved in a symbiotic interaction. References: PMID:18068388, PMID:18941224, PMID:2307127, PMID:28860090 Also known as: disruption by symbiont of host opsonization Relationships: is_a symbiont-mediated perturbation of host defense response [GO:0052031]